{
  "gene_name": "Dapper homolog 1",
  "gene": "UniProtKB:Q9NYF0",
  "term_label": "negative regulation of canonical Wnt signaling pathway",
  "gene_symbol": "DACT1",
  "term_id": "GO:0090090"
}